inhibition of non-skeletal tissue mineralization [GO:0140928] (biological process) Relationships: is a type of tissue homeostasis [GO:0001894] References: PMID:21490328, PMID:30030150 Also known as: inhibition of ectopic tissue mineralization Definition: A homeostatic process involved in the maintenance of non-mineral tissue, by preventing mineralization of non-skeletal tissue.